{
  "term_label": "regulation of inflammatory response",
  "gene": "UniProtKB:P14778",
  "gene_symbol": "IL1R1",
  "term_id": "GO:0050727",
  "gene_name": "Interleukin-1 receptor type 1"
}